{
  "gene_name": "UBA-like domain-containing protein 1",
  "term_id": "UNKNOWN:0002",
  "term_label": "Unknown biological process",
  "gene_symbol": "UBALD1",
  "gene": "UniProtKB:Q8TB05"
}